{
  "gene_name": "Proliferation marker protein Ki-67",
  "gene_symbol": "MKI67",
  "term_id": "GO:0000793",
  "term_label": "condensed chromosome",
  "gene": "UniProtKB:P46013"
}